negative regulation of striated muscle cell apoptotic process [GO:0010664] (biological process) Relationships: is a type of GO:0010656; is a type of regulation of striated muscle cell apoptotic process [GO:0010662]; RO_0002212 striated muscle cell apoptotic process [GO:0010658] Subtypes: GO:0010667 Definition: Any process that decreases the rate or extent of striated muscle cell apoptotic process, a form of programmed cell death induced by external or internal signals that trigger the activity of proteolytic caspases whose actions dismantle a striated muscle cell and result in its death. Also known as: down regulation of striated muscle cell apoptosis, down-regulation of striated muscle cell apoptosis, downregulation of striated muscle cell apoptosis, inhibition of striated muscle cell apoptosis, negative regulation of striated muscle cell apoptosis Sources: GOC:BHF, GOC:dph, GOC:mtg_apoptosis, GOC:rl, GOC:tb